{
  "gene_symbol": "RAB11FIP3",
  "gene_name": "Rab11 family-interacting protein 3",
  "term_label": "midbody",
  "gene": "UniProtKB:O75154",
  "term_id": "GO:0030496"
}